pyrimidine nucleoside monophosphate biosynthetic process [GO:0009130] (biological process) Definition: The chemical reactions and pathways resulting in the formation of pyrimidine nucleoside monophosphate, a compound consisting of a pyrimidine base linked to a ribose or deoxyribose sugar esterified with phosphate on the sugar. Sources: GOC:go_curators, ISBN:0198506732 Also known as: pyrimidine nucleoside monophosphate anabolism, pyrimidine nucleoside monophosphate biosynthesis, pyrimidine nucleoside monophosphate formation, pyrimidine nucleoside monophosphate synthesis Relationships: is a type of GO:0009124; is a type of pyrimidine nucleoside monophosphate metabolic process [GO:0009129] Subtypes: pyrimidine ribonucleoside monophosphate biosynthetic process [GO:0009174], pyrimidine deoxyribonucleoside monophosphate biosynthetic process [GO:0009177]